{
  "gene": "UniProtKB:P06331",
  "term_label": "Unknown cellular component",
  "term_id": "UNKNOWN:0003",
  "gene_symbol": "IGHV4-34",
  "gene_name": "Immunoglobulin heavy variable 4-34"
}